{
  "gene_name": "Neuronal acetylcholine receptor subunit beta-2",
  "gene": "UniProtKB:P17787",
  "term_label": "chemical synaptic transmission",
  "gene_symbol": "CHRNB2",
  "term_id": "GO:0007268"
}